{
  "gene_symbol": "SPOCK2",
  "term_id": "GO:0010810",
  "term_label": "regulation of cell-substrate adhesion",
  "gene": "UniProtKB:Q92563",
  "gene_name": "Testican-2"
}